negative regulation of androgen biosynthetic process [GO:2000180] (BP) Also known as: negative regulation of androgen anabolism, negative regulation of androgen biosynthesis, negative regulation of androgen formation, negative regulation of androgen synthesis Sources: GOC:dph, GOC:yaf Relationships: is a type of negative regulation of steroid biosynthetic process [GO:0010894]; is a type of negative regulation of hormone biosynthetic process [GO:0032353]; negatively regulates GO:0006702 Definition: Any process that stops, prevents, or reduces the frequency, rate or extent of androgen biosynthetic process.